multicellular organism growth [GO:0035264] (biological process) Also known as: body growth Definition: The increase in size or mass of an entire multicellular organism, as opposed to cell growth. Regulation: RO_0002211 by regulation of multicellular organism growth [GO:0040014]; negatively regulated by negative regulation of multicellular organism growth [GO:0040015]; positively regulated by positive regulation of multicellular organism growth [GO:0040018] Sources: GOC:bf, GOC:curators, GOC:dph, GOC:tb Relationships: is_a multicellular organismal process [GO:0032501]; is_a GO:0048589